{
  "gene_symbol": "TIAM2",
  "term_id": "GO:0016020",
  "gene": "UniProtKB:Q8IVF5",
  "gene_name": "Rho guanine nucleotide exchange factor TIAM2",
  "term_label": "membrane"
}